{
  "gene_symbol": "EEF1A1",
  "term_id": "GO:0003924",
  "gene_name": "Elongation factor 1-alpha 1",
  "term_label": "GTPase activity",
  "gene": "UniProtKB:P68104"
}